{
  "gene_name": "Centrosomal protein of 131 kDa",
  "term_label": "centriolar satellite",
  "gene": "UniProtKB:Q9UPN4",
  "gene_symbol": "CEP131",
  "term_id": "GO:0034451"
}